{
  "gene_name": "MAP6 domain-containing protein 1",
  "gene": "UniProtKB:Q9H9H5",
  "term_label": "microtubule",
  "gene_symbol": "MAP6D1",
  "term_id": "GO:0005874"
}